negative regulation of macrophage migration inhibitory factor signaling pathway [GO:2000447] (biological process) Definition: Any process that stops, prevents or reduces the frequency, rate or extent of macrophage migration inhibitory factor signaling pathway. Sources: GOC:obol Also known as: negative regulation of MIF signaling pathway, negative regulation of macrophage migration inhibitory factor signalling pathway Relationships: is a type of negative regulation of cytokine-mediated signaling pathway [GO:0001960]; is a type of regulation of macrophage migration inhibitory factor signaling pathway [GO:2000446]; negatively regulates macrophage migration inhibitory factor signaling pathway [GO:0035691]